UDP-glucuronate dehydrogenase activity [GO:0099618] (molecular function) Also known as: UDP-GlcUA decarboxylase activity, UDP-glucuronic acid dehydrogenase activity Definition: Catalysis of the reaction: UDP-alpha-D-glucuronate + NAD+ = UDP-beta-L-threo-pentopyranos-4-ulose + CO2 + NADH. Sources: RHEA:24702 Relationships: is_a oxidoreductase activity, acting on the CH-OH group of donors, NAD or NADP as acceptor [GO:0016616]